25-hydroxycholecalciferol-23-hydroxylase activity [GO:0062180] (molecular function) References: PMID:22100522, PMID:30205156 Sources: RHEA:46616 Definition: Catalysis of the reaction: calcidiol + 2 H+ + O2 + 2 reduced [adrenodoxin] = (23S)-23,25-dihydroxycalciol + H2O + 2 oxidized [adrenodoxin]. Relationships: is a type of GO:0062179